regulation of MHC class I biosynthetic process [GO:0045343] (biological process) Also known as: regulation of MHC class I anabolism, regulation of MHC class I biosynthesis, regulation of MHC class I formation, regulation of MHC class I synthesis, regulation of major histocompatibility complex class I biosynthesis, regulation of major histocompatibility complex class I biosynthetic process Sources: GOC:go_curators Subtypes: negative regulation of MHC class I biosynthetic process [GO:0045344], GO:0045345 Definition: Any process that modulates the frequency, rate or extent of the chemical reactions and pathways resulting in the formation of MHC class I. Relationships: is a type of regulation of macromolecule biosynthetic process [GO:0010556]; RO_0002211 MHC class I biosynthetic process [GO:0045341]